{
  "term_label": "Unknown molecular function",
  "gene_name": "Spermatogenesis associated 6-like protein",
  "term_id": "UNKNOWN:0001",
  "gene": "UniProtKB:Q8N4H0",
  "gene_symbol": "SPATA6L"
}